CD27 receptor binding [GO:0005175] (molecular function) Definition: Binding to a CD27, a receptor found on the surface of T cells and some B cells and NK cells. Relationships: is a type of tumor necrosis factor receptor superfamily binding [GO:0032813] Sources: GOC:jl, ISBN:0120781859